{
  "gene_name": "Meiosis-specific kinetochore protein",
  "gene_symbol": "MEIKIN",
  "term_label": "meiotic sister chromatid cohesion involved in meiosis I",
  "gene": "UniProtKB:A0A087WXM9",
  "term_id": "GO:0010789"
}